{
  "term_id": "GO:0000977",
  "gene_name": "Transcriptional activator protein Pur-beta",
  "gene": "UniProtKB:Q96QR8",
  "gene_symbol": "PURB",
  "term_label": "RNA polymerase II transcription regulatory region sequence-specific DNA binding"
}